phosphorelay response regulator activity [GO:0000156] (molecular function) Also known as: two-component response regulator activity Definition: Responds to a phosphorelay sensor to initiate a change in cell state or activity. The activity of the response regulator is regulated by transfer of a phosphate from a histidine residue in the sensor, to an aspartate residue in the response regulator. Many but not all response regulators act as transcriptional regulators to elicit a response. References: PMID:10966457, PMID:11842140 Sources: GOC:bf Relationships: is a type of molecular transducer activity [GO:0060089]; is part of GO:0000160